{
  "gene_name": "Stathmin-2",
  "gene_symbol": "STMN2",
  "term_id": "GO:0043005",
  "term_label": "neuron projection",
  "gene": "UniProtKB:Q93045"
}